base J metabolic process [GO:0070580] (biological process) Definition: The chemical reactions and pathways involving base J (beta-D-glucosyl-hydroxymethyluracil), a hypermodified thymidine residue found in the genome of kinetoplastid parasites. This modified base is localized primarily to repetitive DNA, namely the telomeres, and is implicated in the regulation of antigenic variation. The base is synthesized in a two-step pathway. Initially, a thymidine residue in DNA is hydroxylated by a thymidine hydroxylase (TH) to form the intermediate hydroxymethyluracil, which is then glucosylated to form base J. References: PMID:19114062 Also known as: base J metabolism, beta-D-glucosyl-HOMedU metabolic process, beta-D-glucosyl-hydroxymethyluracil metabolism Relationships: is a type of DNA modification [GO:0006304]